{
  "gene": "UniProtKB:Q17RP2",
  "gene_name": "Tigger transposable element-derived protein 6",
  "gene_symbol": "TIGD6",
  "term_label": "nucleus",
  "term_id": "GO:0005634"
}